L-alanine export across the plasma membrane [GO:0140406] (BP) Relationships: is a type of GO:0032973; is a type of L-alanine transmembrane transport [GO:1904557] References: PMID:26073055, PMID:31591285 Definition: The directed movement of L-alanine from inside of a cell, across the plasma membrane and into the extracellular region.